{
  "term_id": "GO:0005549",
  "gene_symbol": "OR8H2",
  "gene": "UniProtKB:Q8N162",
  "gene_name": "Olfactory receptor 8H2",
  "term_label": "odorant binding"
}